apoptotic process involved in luteolysis [GO:0061364] (biological process) Definition: The apoptotic process that contributes to luteolysis. References: PMID:18566128 Sources: GOC:mtg_apoptosis Relationships: is a type of GO:1902742; is part of GO:0001554 Also known as: structural luteolysis, apoptosis involved in luteolysis